L-valine import across plasma membrane [GO:1903805] (biological process) Definition: The directed movement of L-valine from outside of a cell, across the plasma membrane and into the cytosol. References: PMID:23895341 Sources: GOC:TermGenie, GO_REF:0000075 Also known as: L-valine import into cell, valine import Relationships: is a type of amino acid import across plasma membrane [GO:0089718]; is a type of L-valine transmembrane transport [GO:1903785]